{
  "gene_name": "Peptidyl-prolyl cis-trans isomerase A-like 4D",
  "gene": "UniProtKB:F5H284",
  "gene_symbol": "PPIAL4D",
  "term_id": "GO:0003755",
  "term_label": "peptidyl-prolyl cis-trans isomerase activity"
}